protein localization to cytoplasmic stress granule [GO:1903608] (biological process) References: PMID:24755092 Sources: GOC:TermGenie, GO_REF:0000087 Relationships: is a type of GO:0033365 Also known as: protein localization to stress granule, protein localisation in cytoplasmic stress granule, protein localisation to cytoplasmic stress granule, protein localization in cytoplasmic stress granule Definition: A process in which a protein is transported to, or maintained in, a location within a cytoplasmic stress granule.